{
  "term_label": "ATP hydrolysis activity",
  "gene": "UniProtKB:Q2TAC6",
  "gene_name": "Kinesin-like protein KIF19",
  "term_id": "GO:0016887",
  "gene_symbol": "KIF19"
}